sexual sporulation resulting in formation of a multicellular or syncytial spore [GO:0075285] (biological process) Definition: The formation of multicellular or syncytial spore via septations derived from meiosis. A multicellular or syncytial spore is a structure that can be used for dissemination, for survival of adverse conditions because of its heat and desiccation resistance, and/or for reproduction. Relationships: is a type of GO:0034293; is a type of GO:0075283 Sources: GOC:pamgo_curators